{
  "gene_symbol": "EYA1",
  "gene_name": "Eyes absent homolog 1",
  "term_label": "cell differentiation",
  "term_id": "GO:0030154",
  "gene": "UniProtKB:Q99502"
}